{
  "term_label": "mitochondrion",
  "gene_symbol": "MTPAP",
  "term_id": "GO:0005739",
  "gene_name": "Poly(A) RNA polymerase, mitochondrial",
  "gene": "UniProtKB:Q9NVV4"
}